{
  "term_id": "GO:0005886",
  "term_label": "plasma membrane",
  "gene": "UniProtKB:Q96S97",
  "gene_name": "Myeloid-associated differentiation marker",
  "gene_symbol": "MYADM"
}